{
  "term_label": "heteromeric SMAD protein complex",
  "gene_symbol": "SMAD6",
  "gene_name": "Mothers against decapentaplegic homolog 6",
  "gene": "UniProtKB:O43541",
  "term_id": "GO:0071144"
}